{
  "gene_symbol": "WIPI2",
  "gene_name": "WD repeat domain phosphoinositide-interacting protein 2",
  "gene": "UniProtKB:Q9Y4P8",
  "term_id": "GO:0000425",
  "term_label": "pexophagy"
}